{
  "term_id": "GO:0035591",
  "gene_symbol": "DOK5",
  "gene": "UniProtKB:Q9P104",
  "term_label": "signaling adaptor activity",
  "gene_name": "Docking protein 5"
}